{
  "gene_name": "Serine_arginine-rich splicing factor 12",
  "gene_symbol": "SRSF12",
  "term_label": "regulation of alternative mRNA splicing, via spliceosome",
  "gene": "UniProtKB:Q8WXF0",
  "term_id": "GO:0000381"
}